endocrine hormone secretion [GO:0060986] (biological process) Definition: The regulated release of a hormone into the circulatory system. Subtypes: gonadotropin secretion [GO:0032274], inhibin secretion [GO:0032334], GO:0035898, steroid hormone secretion [GO:0035929], juvenile hormone secretion [GO:0045443], corticotropin secretion [GO:0051458], adiponectin secretion [GO:0070162] Sources: GOC:dph Relationships: is a type of GO:0046879; is part of GO:0050886